vacuolar transport [GO:0007034] (biological process) Regulation: regulated by regulation of vacuolar transport [GO:1903335]; negatively regulated by GO:1903336; positively regulated by positive regulation of vacuolar transport [GO:1903337] Definition: The directed movement of substances into, out of or within a vacuole. Subtypes: protein targeting to vacuole [GO:0006623], Golgi to vacuole transport [GO:0006896], endocytosed protein transport to vacuole [GO:0007038], lysosomal transport [GO:0007041], retrograde transport, vacuole to Golgi [GO:0045018], late endosome to vacuole transport [GO:0045324], plastid to vacuole vesicle-mediated transport [GO:1904962] Sources: GOC:ai Relationships: is a type of intracellular transport [GO:0046907]